{
  "term_id": "GO:0005783",
  "term_label": "endoplasmic reticulum",
  "gene_symbol": "TMEM214",
  "gene": "UniProtKB:Q6NUQ4",
  "gene_name": "Transmembrane protein 214"
}